mature natural killer cell chemotaxis [GO:0035782] (biological process) Definition: The directed movement of a mature natural killer cell guided by a specific chemical concentration gradient. Movement may be towards a higher concentration (positive chemotaxis) or towards a lower concentration (negative chemotaxis). A mature natural killer cell is a natural killer cell that is developmentally mature and expresses a variety of inhibitory and activating receptors that recognize MHC class and other stress related molecules. Sources: CL:0000824, GOC:BHF Also known as: activated natural killer cell chemotaxis Relationships: is a type of natural killer cell chemotaxis [GO:0035747]